{
  "term_id": "GO:0005886",
  "term_label": "plasma membrane",
  "gene_symbol": "MRGPRX4",
  "gene_name": "Mas-related G-protein coupled receptor member X4",
  "gene": "UniProtKB:Q96LA9"
}